{
  "gene": "UniProtKB:P31949",
  "gene_name": "Protein S100-A11",
  "term_label": "cytoplasm",
  "term_id": "GO:0005737",
  "gene_symbol": "S100A11"
}